excitatory extracellular ligand-gated monoatomic ion channel activity [GO:0005231] (molecular function) Sources: GOC:mah, ISBN:0323037070 Subtypes: extracellularly ATP-gated monoatomic cation channel activity [GO:0004931], extracellularly glutamate-gated ion channel activity [GO:0005234], extracellularly glycine-gated ion channel activity [GO:0016933], GO:0022848 Definition: Enables the transmembrane transfer of an ion by a channel that opens when a specific extracellular ligand has been bound by the channel complex or one of its constituent parts, where channel opening contributes to an increase in membrane potential. Relationships: is a type of extracellular ligand-gated monoatomic ion channel activity [GO:0005230]; is part of excitatory postsynaptic potential [GO:0060079]